{
  "term_id": "GO:0072542",
  "gene": "UniProtKB:Q5MIZ7",
  "gene_symbol": "PPP4R3B",
  "term_label": "protein phosphatase activator activity",
  "gene_name": "Serine_threonine-protein phosphatase 4 regulatory subunit 3B"
}